ADP transmembrane transporter activity [GO:0015217] (molecular function) Relationships: is a type of GO:0000295; is a type of GO:0005346; is part of GO:0015866 Definition: Enables the transfer of ADP, adenosine diphosphate, from one side of a membrane to the other. Subtypes: ATP:ADP antiporter activity [GO:0005471], ADP:phosphate antiporter activity [GO:0140988] Sources: GOC:ai